{
  "gene": "UniProtKB:Q8IWF7",
  "term_label": "Unknown cellular component",
  "gene_name": "Putative ubiquitin-conjugating enzyme E2 D2-like protein",
  "term_id": "UNKNOWN:0003",
  "gene_symbol": "UBE2DNL"
}